memory T cell proliferation [GO:0061485] (biological process) Relationships: is_a T cell proliferation [GO:0042098] References: PMID:14647273 Sources: GOC:dph Definition: The expansion of a memory T cell population by cell division.